serum response element binding [GO:0010736] (molecular function) Definition: Binding to a serum response element (SRE), a short sequence with dyad symmetry found in the promoters of some of the cellular immediate-early genes, regulated by serum. Sources: GOC:BHF, GOC:dph, GOC:rl, GOC:tb Relationships: is a type of RNA polymerase II cis-regulatory region sequence-specific DNA binding [GO:0000978]